{
  "gene_symbol": "FAM228A",
  "term_label": "Unknown molecular function",
  "term_id": "UNKNOWN:0001",
  "gene_name": "Protein FAM228A",
  "gene": "UniProtKB:Q86W67"
}